{
  "gene_symbol": "A8MUA0",
  "term_id": "UNKNOWN:0001",
  "term_label": "Unknown molecular function",
  "gene": "UniProtKB:A8MUA0",
  "gene_name": "Putative UPF0607 protein ENSP00000381514"
}